{
  "gene": "UniProtKB:P15382",
  "gene_symbol": "KCNE1",
  "gene_name": "Potassium voltage-gated channel subfamily E member 1",
  "term_id": "GO:0008076",
  "term_label": "voltage-gated potassium channel complex"
}